response to vitamin B3 [GO:0033552] (biological process) Definition: Any process that results in a change in state or activity of a cell or an organism (in terms of movement, secretion, enzyme production, gene expression, etc.) as a result of a vitamin B3 stimulus. Sources: GOC:sl Also known as: response to niacin, response to nicotinamide Relationships: is a type of response to vitamin [GO:0033273] Subtypes: cellular response to vitamin B3 [GO:0071303]